amylin receptor complex [GO:1903440] (cellular component) Definition: A protein complex which is capable of amylin receptor activity. References: PMID:10871296, PMID:12037140, PMID:18687416 Sources: GOC:TermGenie, GOC:bhm, GO_REF:0000088 Relationships: is_a GO:1903439 Subtypes: amylin receptor complex 1 [GO:0150056], amylin receptor complex 2 [GO:0150057], GO:0150058